{
  "gene_name": "Phospholipase A and acyltransferase 5",
  "gene_symbol": "PLAAT5",
  "term_id": "GO:0004623",
  "term_label": "phospholipase A2 activity",
  "gene": "UniProtKB:Q96KN8"
}